NADP+ binding [GO:0070401] (molecular function) Definition: Binding to the oxidized form, NADP+, of nicotinamide-adenine dinucleotide phosphate, a coenzyme involved in many redox and biosynthetic reactions. Also known as: NADP (oxidized) binding, oxidized NADP binding, oxidized nicotinamide adenine dinucleotide phosphate binding, NADP binding Relationships: is a type of anion binding [GO:0043168]; is a type of NADP binding [GO:0050661] Sources: GOC:mah